{
  "gene": "UniProtKB:Q96RI1",
  "term_id": "GO:0042632",
  "gene_symbol": "NR1H4",
  "gene_name": "Bile acid receptor",
  "term_label": "cholesterol homeostasis"
}